negative regulation of cardiac cell fate specification [GO:2000044] (biological process) Definition: Any process that stops, prevents, or reduces the frequency, rate or extent of cardiac cell fate specification. Subtypes: negative regulation of cardioblast cell fate specification [GO:0009997] Sources: GOC:BHF Relationships: is a type of negative regulation of cell fate specification [GO:0009996]; is a type of negative regulation of cardiocyte differentiation [GO:1905208]; is_a regulation of cardiac cell fate specification [GO:2000043]; negatively regulates cardiac cell fate specification [GO:0060912]